presynaptic active zone [GO:0048786] (cellular component) Definition: A specialized region of the plasma membrane and cell cortex of a presynaptic neuron; encompasses a region of the plasma membrane where synaptic vesicles dock and fuse, and a specialized cortical cytoskeletal matrix. Also known as: pre-synaptic active zone, presynaptic specialization, pre-synaptic active zone component Relationships: is a type of cellular anatomical structure [GO:0110165]; is part of presynapse [GO:0098793] References: PMID:3152289 Sources: GOC:dh, GOC:dl, GOC:ef, GOC:jid, GOC:pr